{
  "gene_name": "High affinity cAMP-specific and IBMX-insensitive 3',5'-cyclic phosphodiesterase 8A",
  "term_id": "GO:0141162",
  "term_label": "negative regulation of cAMP/PKA signal transduction",
  "gene_symbol": "PDE8A",
  "gene": "UniProtKB:O60658"
}